{
  "gene": "UniProtKB:Q9Y210",
  "gene_name": "Short transient receptor potential channel 6",
  "term_id": "GO:0034703",
  "term_label": "cation channel complex",
  "gene_symbol": "TRPC6"
}